renal vesicle induction [GO:0072034] (biological process) Sources: GOC:mtg_kidney_jan10 Also known as: nephron induction, positive regulation of nephron formation Definition: Signaling at short range between cells of the ureteric bud terminus and the kidney mesenchyme that positively regulates the formation of the renal vesicle. Relationships: is a type of developmental induction [GO:0031128]; is a type of positive regulation of kidney development [GO:0090184]; is a type of positive regulation of animal organ morphogenesis [GO:0110110]; is a type of positive regulation of morphogenesis of an epithelium [GO:1905332]; RO_0002213 renal vesicle formation [GO:0072033] Subtypes: mesonephric renal vesicle induction [GO:0061294], GO:0072094